cluster of actin-based cell projections [GO:0098862] (cellular component) Sources: GOC:dos Definition: A cell part consisting of multiple, closely packed actin-based cell projections. Subtypes: brush border [GO:0005903], stereocilium bundle [GO:0032421], GO:0151001 Relationships: is a type of cellular anatomical structure [GO:0110165]; has part actin-based cell projection [GO:0098858]